{
  "gene_name": "Histatin-1",
  "term_label": "mitochondrion",
  "gene": "UniProtKB:P15515",
  "gene_symbol": "HTN1",
  "term_id": "GO:0005739"
}